{
  "term_id": "UNKNOWN:0003",
  "gene_symbol": "A8MV72",
  "gene": "UniProtKB:A8MV72",
  "gene_name": "Putative UPF0607 protein ENSP00000382826",
  "term_label": "Unknown cellular component"
}